positive regulation of protein folding [GO:1903334] (biological process) Sources: GOC:TermGenie, GOC:vw, GO_REF:0000058 Relationships: is a type of GO:0048522; is a type of regulation of protein folding [GO:1903332]; positively regulates protein folding [GO:0006457] Subtypes: positive regulation of protein refolding [GO:1904592] Definition: Any process that activates or increases the frequency, rate or extent of protein folding. Also known as: up regulation of protein folding, up-regulation of protein folding, upregulation of protein folding, activation of alpha-tubulin folding, activation of beta-tubulin folding, activation of chaperonin-mediated tubulin folding, activation of protein folding, positive regulation of alpha-tubulin folding, positive regulation of beta-tubulin folding, positive regulation of chaperonin-mediated tubulin folding, up regulation of alpha-tubulin folding, up regulation of beta-tubulin folding, up regulation of chaperonin-mediated tubulin folding, up-regulation of alpha-tubulin folding, up-regulation of beta-tubulin folding, up-regulation of chaperonin-mediated tubulin folding, upregulation of alpha-tubulin folding, upregulation of beta-tubulin folding, upregulation of chaperonin-mediated tubulin folding, activation of chaperone activity, activation of chaperonin ATPase activity, activation of co-chaperone activity, activation of co-chaperonin activity, activation of glycoprotein-specific chaperone activity, activation of non-chaperonin molecular chaperone ATPase activity, activation of protein complex assembly, multichaperone pathway, positive regulation of chaperone activity, positive regulation of chaperonin ATPase activity, positive regulation of co-chaperone activity, positive regulation of co-chaperonin activity, positive regulation of glycoprotein-specific chaperone activity, positive regulation of non-chaperonin molecular chaperone ATPase activity, positive regulation of protein complex assembly, multichaperone pathway, up regulation of chaperone activity, up regulation of chaperonin ATPase activity, up regulation of co-chaperone activity, up regulation of co-chaperonin activity, up regulation of glycoprotein-specific chaperone activity, up regulation of non-chaperonin molecular chaperone ATPase activity, up regulation of protein complex assembly, multichaperone pathway, up-regulation of chaperone activity, up-regulation of chaperonin ATPase activity, up-regulation of co-chaperone activity, up-regulation of co-chaperonin activity, up-regulation of glycoprotein-specific chaperone activity, up-regulation of non-chaperonin molecular chaperone ATPase activity, up-regulation of protein complex assembly, multichaperone pathway, upregulation of chaperone activity, upregulation of chaperonin ATPase activity, upregulation of co-chaperone activity, upregulation of co-chaperonin activity, upregulation of glycoprotein-specific chaperone activity, upregulation of non-chaperonin molecular chaperone ATPase activity, upregulation of protein complex assembly, multichaperone pathway